{
  "gene_symbol": "CHD1L",
  "gene_name": "Chromodomain-helicase-DNA-binding protein 1-like",
  "term_id": "GO:0005634",
  "term_label": "nucleus",
  "gene": "UniProtKB:Q86WJ1"
}